skeletal muscle organ development [GO:0060538] (biological process) Relationships: is a type of muscle organ development [GO:0007517] Sources: GOC:dph Subtypes: extraocular skeletal muscle development [GO:0002074], somitomeric trunk muscle development [GO:0002075], diaphragm development [GO:0060539] Definition: The progression of a skeletal muscle organ over time from its initial formation to its mature state. A skeletal muscle organ includes the skeletal muscle tissue and its associated connective tissue.